{
  "gene": "UniProtKB:P40617",
  "term_label": "cytoplasm",
  "gene_symbol": "ARL4A",
  "term_id": "GO:0005737",
  "gene_name": "ADP-ribosylation factor-like protein 4A"
}